{
  "gene_name": "Probable ribonuclease ZC3H12D",
  "gene_symbol": "ZC3H12D",
  "term_id": "GO:0005634",
  "gene": "UniProtKB:A2A288",
  "term_label": "nucleus"
}